{
  "term_label": "Unknown biological process",
  "gene": "UniProtKB:Q9NYJ1",
  "gene_name": "Cytochrome c oxidase assembly factor 4 homolog, mitochondrial",
  "term_id": "UNKNOWN:0002",
  "gene_symbol": "COA4"
}